mannan polymerase II complex [GO:0140497] (cellular component) Definition: A complex with alpha-(1->6)-mannosyltransferase activity, located in the cis Golgi membrane; adds mannan to N-linked glycans on proteins as part of the elongation of alpha 1,6-linked Man backbone. In S. cerevisiae, contains Mnn9p, Anp1p, Mnn10p, Mnn11p, and Hoc1p. References: PMID:9430634 Relationships: is a type of GO:0000136